urethra development [GO:0061068] (biological process) Subtypes: male urethra development [GO:0061069], female urethra development [GO:0061070] Relationships: is a type of GO:0048513; is part of renal system development [GO:0072001] Sources: GOC:dph Definition: The progression of the urethra over time from its initial formation to the mature structure. The urethra is a renal system organ that carries urine from the bladder to outside the body.